triglyceride-rich plasma lipoprotein particle [GO:0034385] (cellular component) Also known as: triglyceride-rich lipoprotein particle, triacylglycerol-rich lipoprotein particle Sources: GOC:BHF, GOC:mah, GOC:rl Subtypes: very-low-density lipoprotein particle [GO:0034361], GO:0034363 Relationships: is a type of plasma lipoprotein particle [GO:0034358] Definition: A plasma lipoprotein particle that has a hydrophobic core enriched in triglycerides surrounded by an amphipathic monolayer of phospholipids, cholesterol and apolipoproteins. Triglyceride-rich lipoprotein particles transport lipids, which are non-covalently associated with the particles, in the blood.